{
  "term_label": "plasma membrane",
  "gene": "UniProtKB:P25116",
  "gene_symbol": "F2R",
  "gene_name": "Proteinase-activated receptor 1",
  "term_id": "GO:0005886"
}